{
  "gene": "UniProtKB:Q9P2F8",
  "gene_name": "Signal-induced proliferation-associated 1-like protein 2",
  "term_id": "UNKNOWN:0002",
  "gene_symbol": "SIPA1L2",
  "term_label": "Unknown biological process"
}